cytokine binding [GO:0019955] (molecular function) Definition: Binding to a cytokine, any of a group of proteins that function to control the survival, growth and differentiation of tissues and cells, and which have autocrine and paracrine activity. Sources: GOC:ai, GOC:bf, ISBN:0198599471 Also known as: IL binding, interleukin binding Relationships: is a type of protein binding [GO:0005515] Subtypes: GO:0002113, chemokine binding [GO:0019956], GO:0019961, interleukin-1 binding [GO:0019966], interleukin-10 binding [GO:0019969], GO:0019970, interleukin-12 binding [GO:0019972], interleukin-13 binding [GO:0019973], interleukin-17 binding [GO:0019975], GO:0019976, interleukin-21 binding [GO:0019977], interleukin-3 binding [GO:0019978], interleukin-4 binding [GO:0019979], interleukin-5 binding [GO:0019980], interleukin-6 binding [GO:0019981], interleukin-7 binding [GO:0019982], interleukin-9 binding [GO:0019983], macrophage migration inhibitory factor binding [GO:0035718], BMP binding [GO:0036122], GO:0042007, interleukin-15 binding [GO:0042009], interleukin-16 binding [GO:0042011], GO:0042013, interleukin-20 binding [GO:0042015], interleukin-22 binding [GO:0042017], interleukin-23 binding [GO:0042019], granulocyte macrophage colony-stimulating factor complex binding [GO:0042021], tumor necrosis factor binding [GO:0043120], GO:0045510, interleukin-26 binding [GO:0045512], transforming growth factor beta binding [GO:0050431], granulocyte colony-stimulating factor binding [GO:0051916], GO:0070119, high mobility group box 1 binding [GO:0070379], interleukin-35 binding [GO:0070746]